{
  "gene_name": "U3 small nucleolar RNA-associated protein 4 homolog",
  "term_id": "GO:0032040",
  "gene": "UniProtKB:Q969X6",
  "term_label": "small-subunit processome",
  "gene_symbol": "UTP4"
}